negative regulation of ergot alkaloid biosynthetic process [GO:1900823] (biological process) Definition: Any process that stops, prevents or reduces the frequency, rate or extent of ergot alkaloid biosynthetic process. Sources: GOC:TermGenie, GOC:di Subtypes: negative regulation of chanoclavine-I aldehyde biosynthetic process [GO:1900647], negative regulation of fumigaclavine C biosynthetic process [GO:1900838] Also known as: down regulation of ergot alkaloid anabolism, down regulation of ergot alkaloid biosynthesis, down regulation of ergot alkaloid biosynthetic process, down regulation of ergot alkaloid formation, down regulation of ergot alkaloid synthesis, down-regulation of ergot alkaloid anabolism, down-regulation of ergot alkaloid biosynthesis, down-regulation of ergot alkaloid biosynthetic process, down-regulation of ergot alkaloid formation, down-regulation of ergot alkaloid synthesis, downregulation of ergot alkaloid anabolism, downregulation of ergot alkaloid biosynthesis, downregulation of ergot alkaloid biosynthetic process, downregulation of ergot alkaloid formation, downregulation of ergot alkaloid synthesis, inhibition of ergot alkaloid anabolism, inhibition of ergot alkaloid biosynthesis, inhibition of ergot alkaloid formation, inhibition of ergot alkaloid synthesis, negative regulation of ergot alkaloid anabolism, negative regulation of ergot alkaloid biosynthesis, negative regulation of ergot alkaloid formation, negative regulation of ergot alkaloid synthesis, inhibition of ergot alkaloid biosynthetic process Relationships: is a type of GO:1900377; is a type of regulation of ergot alkaloid biosynthetic process [GO:1900822]; negatively regulates ergot alkaloid biosynthetic process [GO:0035837]